{
  "gene": "UniProtKB:Q13459",
  "gene_name": "Unconventional myosin-IXb",
  "term_label": "microfilament motor activity",
  "gene_symbol": "MYO9B",
  "term_id": "GO:0000146"
}